{
  "gene": "UniProtKB:P49458",
  "term_id": "GO:0006614",
  "gene_symbol": "SRP9",
  "term_label": "SRP-dependent cotranslational protein targeting to membrane",
  "gene_name": "Signal recognition particle 9 kDa protein"
}